{
  "term_id": "UNKNOWN:0001",
  "gene": "UniProtKB:Q8WZ26",
  "gene_symbol": "PP6455",
  "gene_name": "Putative uncharacterized protein PP6455",
  "term_label": "Unknown molecular function"
}